phytol kinase activity [GO:0010276] (molecular function) Relationships: is a type of kinase activity [GO:0016301] Definition: Catalysis of the reaction: phytol + CTP = phytyl monophosphate + CDP + H+. Sources: RHEA:38055